{
  "gene": "UniProtKB:Q969E3",
  "gene_symbol": "UCN3",
  "term_id": "GO:0007189",
  "gene_name": "Urocortin-3",
  "term_label": "adenylate cyclase-activating G protein-coupled receptor signaling pathway"
}